erythrocyte differentiation [GO:0030218] (biological process) Regulation: regulated by regulation of erythrocyte differentiation [GO:0045646]; negatively regulated by negative regulation of erythrocyte differentiation [GO:0045647]; positively regulated by positive regulation of erythrocyte differentiation [GO:0045648] Sources: GOC:mah Subtypes: enucleate erythrocyte differentiation [GO:0043353], GO:0043363, definitive erythrocyte differentiation [GO:0060318], primitive erythrocyte differentiation [GO:0060319] Relationships: is a type of myeloid cell differentiation [GO:0030099]; BFO_0000050 erythrocyte homeostasis [GO:0034101] Definition: The process in which a myeloid precursor cell acquires specializes features of an erythrocyte. Also known as: RBC differentiation, erythrocyte cell differentiation, erythropoiesis, red blood cell differentiation